{
  "gene": "UniProtKB:Q9H4S2",
  "gene_symbol": "GSX1",
  "term_label": "nucleus",
  "term_id": "GO:0005634",
  "gene_name": "GS homeobox 1"
}